allantoin assimilation pathway [GO:0009442] (BP) Definition: The pathways by which allantoin is processed and converted to ureidoglycolate, and then into metabolically useful substrates. E. coli are able to utilize allantoin as a sole nitrogen source under anaerobic conditions by converting it to ureidoglycolate; this may be further metabolized to produce glyoxylate and thence 3-phosphoglycerate, or alternatively oxidized to oxolureate, which can converted into oxamate and carbamoylphosphate. This may then be further metabolized to CO2, NH4+ and ATP. Relationships: is a type of GO:0000256 Sources: MetaCyc:PWY0-41 Also known as: allantoin catabolic process via ureidoglycolate, allantoin catabolism via ureidoglycolate, allantoin degradation pathway